{
  "gene_symbol": "CEP135",
  "term_label": "centriole",
  "term_id": "GO:0005814",
  "gene": "UniProtKB:Q66GS9",
  "gene_name": "Centrosomal protein of 135 kDa"
}